positive regulation of mitochondrial fusion [GO:0010636] (biological process) Relationships: is a type of regulation of mitochondrial fusion [GO:0010635]; is a type of positive regulation of organelle organization [GO:0010638]; is a type of positive regulation of developmental process [GO:0051094]; positively regulates mitochondrial fusion [GO:0008053] Definition: Any process that increases the frequency, rate or extent of merging of two or more mitochondria within a cell to form a single compartment. Sources: GOC:dph, GOC:tb